{
  "term_id": "UNKNOWN:0003",
  "gene_symbol": "TEX50",
  "gene": "UniProtKB:A0A1B0GTY4",
  "gene_name": "Testis-expressed protein 50",
  "term_label": "Unknown cellular component"
}